{
  "term_label": "NAD+ poly-ADP-ribosyltransferase activity",
  "gene": "UniProtKB:Q9Y6F1",
  "term_id": "GO:0003950",
  "gene_name": "Protein mono-ADP-ribosyltransferase PARP3",
  "gene_symbol": "PARP3"
}